{
  "gene_symbol": "LAS2",
  "gene_name": "Lung adenoma susceptibility protein 2",
  "term_id": "UNKNOWN:0001",
  "term_label": "Unknown molecular function",
  "gene": "UniProtKB:Q8IYD9"
}